{
  "gene": "UniProtKB:Q96JT2",
  "gene_symbol": "SLC45A3",
  "term_id": "UNKNOWN:0002",
  "gene_name": "Solute carrier family 45 member 3",
  "term_label": "Unknown biological process"
}